3,4-dihydroxybenzoate catabolic process [GO:0019619] (biological process) Definition: The chemical reactions and pathways resulting in the breakdown of 3,4-dihydroxybenzoate. Relationships: is a type of catechol-containing compound catabolic process [GO:0019614]; is a type of 3,4-dihydroxybenzoate metabolic process [GO:0046278]; is a type of GO:0072329 Sources: GOC:ai Subtypes: GO:0019617, protocatechuate catabolic process, ortho-cleavage [GO:0019618] Also known as: protocatechuate breakdown, protocatechuate catabolic process, protocatechuate catabolism, protocatechuate degradation